{
  "term_label": "lysozyme activity",
  "term_id": "GO:0003796",
  "gene": "UniProtKB:Q6UWQ5",
  "gene_symbol": "LYZL1",
  "gene_name": "Lysozyme-like protein 1"
}